{
  "gene_name": "GTP-binding protein SAR1b",
  "term_label": "regulation of COPII vesicle coating",
  "gene_symbol": "SAR1B",
  "gene": "UniProtKB:Q9Y6B6",
  "term_id": "GO:0003400"
}